{
  "term_label": "siderophore biosynthetic process",
  "term_id": "GO:0019290",
  "gene_symbol": "BDH2",
  "gene_name": "Dehydrogenase_reductase SDR family member 6",
  "gene": "UniProtKB:Q9BUT1"
}